{
  "term_id": "GO:0051056",
  "gene": "UniProtKB:Q14CB8",
  "gene_name": "Rho GTPase-activating protein 19",
  "term_label": "regulation of small GTPase mediated signal transduction",
  "gene_symbol": "ARHGAP19"
}